positive regulation of protein localization to endoplasmic reticulum [GO:1905552] (biological process) Also known as: positive regulation of protein localisation in endoplasmic reticulum, positive regulation of protein localization in ER, positive regulation of protein localization in endoplasmic reticulum, up regulation of protein localisation in endoplasmic reticulum, up regulation of protein localization in ER, up regulation of protein localization in endoplasmic reticulum, up regulation of protein localization to endoplasmic reticulum, up-regulation of protein localisation in endoplasmic reticulum, up-regulation of protein localization in ER, up-regulation of protein localization in endoplasmic reticulum, up-regulation of protein localization to endoplasmic reticulum, upregulation of protein localisation in endoplasmic reticulum, upregulation of protein localization in ER, upregulation of protein localization in endoplasmic reticulum, upregulation of protein localization to endoplasmic reticulum, activation of protein localisation in endoplasmic reticulum, activation of protein localization in ER, activation of protein localization in endoplasmic reticulum, activation of protein localization to endoplasmic reticulum Relationships: is a type of positive regulation of protein localization [GO:1903829]; is a type of regulation of protein localization to endoplasmic reticulum [GO:1905550]; positively regulates protein localization to endoplasmic reticulum [GO:0070972] References: PMID:22768340 Sources: GOC:TermGenie, GO_REF:0000058 Definition: Any process that activates or increases the frequency, rate or extent of protein localization to endoplasmic reticulum.